proximal convoluted tubule segment 1 cell fate commitment [GO:0072154] (biological process) Also known as: S1 cell fate commitment Definition: The process in which the developmental fate of a cell becomes restricted such that it will develop into an S1 cell in the kidney. Relationships: is a type of cell fate commitment [GO:0045165]; is part of proximal convoluted tubule segment 1 cell differentiation [GO:0072062] Sources: GOC:bf, GOC:mtg_kidney_jan10